circadian sleep/wake cycle, wakefulness [GO:0042746] (biological process) Definition: The part of the circadian sleep/wake cycle where the organism is not asleep. References: PMID:12575468 Sources: GOC:jl Relationships: is a type of circadian sleep/wake cycle process [GO:0022410] Regulation: regulated by regulation of circadian sleep/wake cycle, wakefulness [GO:0010840]; positively regulated by positive regulation of circadian sleep/wake cycle, wakefulness [GO:0010841]; negatively regulated by negative regulation of circadian sleep/wake cycle, wakefulness [GO:1904326]